{
  "gene_name": "Protein LSM12",
  "term_id": "UNKNOWN:0001",
  "gene_symbol": "LSM12",
  "gene": "UniProtKB:Q3MHD2",
  "term_label": "Unknown molecular function"
}